{
  "gene_symbol": "COBL",
  "gene": "UniProtKB:O75128",
  "term_label": "actin filament",
  "term_id": "GO:0005884",
  "gene_name": "Protein cordon-bleu"
}